{
  "term_id": "UNKNOWN:0001",
  "gene_name": "Noelin-3",
  "term_label": "Unknown molecular function",
  "gene_symbol": "OLFM3",
  "gene": "UniProtKB:Q96PB7"
}